ribosomal subunit export from nucleus [GO:0000054] (biological process) Regulation: regulated by regulation of ribosomal subunit export from nucleus [GO:2000200]; negatively regulated by negative regulation of ribosomal subunit export from nucleus [GO:2000201]; positively regulated by GO:2000202 Also known as: ribosomal subunit export from cell nucleus, ribosomal subunit export out of nucleus, ribosomal subunit transport from nucleus to cytoplasm, ribosomal subunit-nucleus export, ribosome export from nucleus Sources: GOC:ai Definition: The directed movement of a ribosomal subunit from the nucleus into the cytoplasm. Subtypes: GO:0000055, GO:0000056 Relationships: is a type of ribosome localization [GO:0033750]; is a type of nuclear export [GO:0051168]; is a type of establishment of organelle localization [GO:0051656]; is part of ribosome biogenesis [GO:0042254]